{
  "gene_symbol": "SUSD3",
  "gene": "UniProtKB:Q96L08",
  "term_id": "UNKNOWN:0001",
  "gene_name": "Sushi domain-containing protein 3",
  "term_label": "Unknown molecular function"
}